metacyclogenesis [GO:0140384] (biological process) Relationships: is a type of GO:0044114 References: PMID:12152483, PMID:21514274, PMID:2659372, PMID:29091711, PMID:29409544 Definition: The morphological, biochemical and genetic changes that induce the differentiation of non-pathogenic parasites into pathogenic metacyclic parasites in the Trypanosomatidae species. The pathogenic parasites are known as metacyclic trypomastigotes in Trypanosoma and metacyclic promastigotes in Leishmania.